manganese ion transmembrane transport [GO:0071421] (biological process) Relationships: is a type of GO:0006828; is a type of GO:0098655 Definition: A process in which a manganese ion is transported from one side of a membrane to the other by means of some agent such as a transporter or pore. Sources: GOC:mah Subtypes: manganese ion export across plasma membrane [GO:0140048], GO:0140967, mitochondrial manganese ion transmembrane transport [GO:1990540] Also known as: manganese ion membrane transport, transmembrane manganese transport Note: Note that this term is not intended for use in annotating lateral movement within membranes.